{
  "term_id": "GO:0005829",
  "gene": "UniProtKB:Q86VQ6",
  "term_label": "cytosol",
  "gene_symbol": "TXNRD3",
  "gene_name": "Thioredoxin reductase 3"
}